vascular endothelial growth factor binding [GO:0038085] (molecular function) Relationships: is a type of growth factor binding [GO:0019838] References: PMID:17470632 Also known as: VEGF binding Definition: Binding to a vascular endothelial growth factor.